{
  "term_id": "UNKNOWN:0003",
  "gene": "UniProtKB:Q5QFB9",
  "gene_symbol": "PAPPA-AS1",
  "gene_name": "Protein PAPPAS",
  "term_label": "Unknown cellular component"
}